{
  "gene": "UniProtKB:Q9NZH7",
  "term_label": "inflammatory response",
  "gene_symbol": "IL36B",
  "term_id": "GO:0006954",
  "gene_name": "Interleukin-36 beta"
}